{
  "term_label": "transport along microtubule",
  "gene_name": "Cytoplasmic dynein 1 intermediate chain 2",
  "gene": "UniProtKB:Q13409",
  "gene_symbol": "DYNC1I2",
  "term_id": "GO:0010970"
}